{
  "gene": "UniProtKB:P05090",
  "gene_symbol": "APOD",
  "term_label": "cytoplasm",
  "gene_name": "Apolipoprotein D",
  "term_id": "GO:0005737"
}